{
  "gene": "UniProtKB:H0Y354",
  "term_id": "UNKNOWN:0002",
  "gene_symbol": "FAM72C",
  "gene_name": "Protein FAM72C",
  "term_label": "Unknown biological process"
}